oculomotor nerve morphogenesis [GO:0021622] (biological process) Also known as: CN III morphogenesis Relationships: is a type of GO:0021602; is part of oculomotor nerve development [GO:0021557] Definition: The process in which the anatomical structure of the oculomotor nerve is generated and organized. This motor nerve innervates all extraocular muscles except the superior oblique and the lateral rectus muscles. The superior division supplies the levator palpebrae superioris and superior rectus muscles. The inferior division supplies the medial rectus, inferior rectus and inferior oblique muscles. This nerve also innervates the striated muscles of the eyelid. Pupillary constriction and lens movement are mediated by this nerve for near vision. In the orbit the inferior division sends branches that enter the ciliary ganglion where they form functional contacts (synapses) with the ganglion cells. The ganglion cells send nerve fibers into the back of the eye where they travel to ultimately innervate the ciliary muscle and the constrictor pupillae muscle. Sources: GOC:cls, GOC:dgh, GOC:dph, GOC:jid, GO_REF:0000021